{
  "gene": "UniProtKB:Q5T6F0",
  "gene_symbol": "DCAF12",
  "gene_name": "DDB1- and CUL4-associated factor 12",
  "term_label": "Unknown molecular function",
  "term_id": "UNKNOWN:0001"
}